{
  "term_id": "GO:0005886",
  "gene_symbol": "LHCGR",
  "gene_name": "Lutropin-choriogonadotropic hormone receptor",
  "gene": "UniProtKB:P22888",
  "term_label": "plasma membrane"
}